{
  "term_label": "Unknown molecular function",
  "gene_symbol": "PNMA2",
  "gene_name": "Paraneoplastic antigen Ma2",
  "gene": "UniProtKB:Q9UL42",
  "term_id": "UNKNOWN:0001"
}